{
  "gene_name": "25-hydroxyvitamin D-1 alpha hydroxylase, mitochondrial",
  "gene": "UniProtKB:O15528",
  "term_label": "calcidiol 1-monooxygenase activity",
  "term_id": "GO:0004498",
  "gene_symbol": "CYP27B1"
}